{
  "gene_symbol": "NPFF",
  "term_label": "perikaryon",
  "gene": "UniProtKB:O15130",
  "gene_name": "Pro-FMRFamide-related neuropeptide FF",
  "term_id": "GO:0043204"
}